{
  "gene": "UniProtKB:A0A494C086",
  "gene_symbol": "SPDYE21",
  "term_id": "GO:0019901",
  "term_label": "protein kinase binding",
  "gene_name": "Putative speedy protein E21"
}